negative regulation of (R)-carnitine transmembrane transport [GO:1902273] (BP) Also known as: down regulation of (R)-carnitine transmembrane transport, down-regulation of (R)-carnitine transmembrane transport, downregulation of (R)-carnitine transmembrane transport, inhibition of (R)-carnitine transmembrane transport Definition: Any process that stops, prevents or reduces the frequency, rate or extent of (R)-carnitine transmembrane transport. References: PMID:23755272 Sources: GOC:TermGenie Relationships: is a type of negative regulation of transmembrane transport [GO:0034763]; is_a regulation of (R)-carnitine transmembrane transport [GO:1902272]; negatively regulates GO:1902270